type 1 proteinase activated receptor binding [GO:0031872] (molecular function) Definition: Binding to a type 1 proteinase activated receptor. Also known as: thrombin receptor binding, type 1 proteinase activated receptor ligand Relationships: is a type of GO:0031871 Sources: GOC:mah, GOC:nln